negative regulation of immune system process [GO:0002683] (biological process) Also known as: down regulation of immune system process, down-regulation of immune system process, downregulation of immune system process, inhibition of immune system process Subtypes: negative regulation of antigen processing and presentation [GO:0002578], negative regulation of tolerance induction [GO:0002644], GO:0002686, negative regulation of leukocyte activation [GO:0002695], negative regulation of immune effector process [GO:0002698], negative regulation of mast cell apoptotic process [GO:0033026], negative regulation of erythrocyte clearance [GO:0034107], negative regulation of toll-like receptor signaling pathway [GO:0034122], negative regulation of toll-like receptor 1 signaling pathway [GO:0034132], negative regulation of toll-like receptor 2 signaling pathway [GO:0034136], GO:0034144, GO:0034148, negative regulation of toll-like receptor 6 signaling pathway [GO:0034152], negative regulation of toll-like receptor 10 signaling pathway [GO:0034168], negative regulation of hemocyte proliferation [GO:0035207], negative regulation of cytoplasmic pattern recognition receptor signaling pathway [GO:0039532], negative regulation of hemocyte differentiation [GO:0045611], negative regulation of immune response [GO:0050777], negative regulation of antigen receptor-mediated signaling pathway [GO:0050858], negative regulation of peptidoglycan recognition protein signaling pathway [GO:0061060], GO:0070236, negative regulation of activated T cell autonomous cell death [GO:0070240], negative regulation of hemopoiesis [GO:1903707], negative regulation of toll-like receptor 15 signaling pathway [GO:2000441], negative regulation of T cell costimulation [GO:2000524] Definition: Any process that stops, prevents, or reduces the frequency, rate, or extent of an immune system process. Relationships: is a type of regulation of immune system process [GO:0002682]; is a type of negative regulation of biological process [GO:0048519]; negatively regulates immune system process [GO:0002376] Sources: GOC:add